DN2 thymocyte differentiation [GO:1904155] (biological process) References: PMID:25398325 Sources: GOC:TermGenie, GOC:dph, GO_REF:0000086 Definition: The process in which a relatively unspecialized cell acquires the specialized features of a DN2 thymocyte. A DN2 thymocyte is a CD4-,CD8- thymocyte that is also CD44+,CD25-. Relationships: is a type of GO:0033077